{
  "gene_name": "Myeloid-derived growth factor",
  "term_label": "extracellular space",
  "gene": "UniProtKB:Q969H8",
  "gene_symbol": "MYDGF",
  "term_id": "GO:0005615"
}